detection of symbiotic fungus [GO:0009603] (biological process) Relationships: is_a detection of symbiont [GO:0009602]; is a type of response to symbiotic fungus [GO:0009610]; is a type of detection of fungus [GO:0016046] Also known as: detection of symbiotic fungi, perception of symbiotic fungi, perception of symbiotic fungus Sources: GOC:hb, ISBN:0198506732 Definition: The series of events in which a stimulus from a symbiotic fungus, a fungus living in close physical association with another organism, is received and converted into a molecular signal.